{
  "gene_name": "Large ribosomal subunit protein uL24",
  "term_label": "structural constituent of ribosome",
  "gene": "UniProtKB:P61254",
  "term_id": "GO:0003735",
  "gene_symbol": "RPL26"
}